{
  "gene_name": "Zinc finger protein 547",
  "term_id": "GO:0006357",
  "gene": "UniProtKB:Q8IVP9",
  "gene_symbol": "ZNF547",
  "term_label": "regulation of transcription by RNA polymerase II"
}